{
  "term_label": "cytoskeleton",
  "gene_name": "Cdc42 effector protein 4",
  "gene_symbol": "CDC42EP4",
  "term_id": "GO:0005856",
  "gene": "UniProtKB:Q9H3Q1"
}